{
  "term_id": "GO:0000978",
  "gene": "UniProtKB:P85037",
  "term_label": "RNA polymerase II cis-regulatory region sequence-specific DNA binding",
  "gene_name": "Forkhead box protein K1",
  "gene_symbol": "FOXK1"
}